{
  "gene": "UniProtKB:P28222",
  "term_id": "GO:0030425",
  "gene_name": "5-hydroxytryptamine receptor 1B",
  "term_label": "dendrite",
  "gene_symbol": "HTR1B"
}